{
  "gene_symbol": "ZNF541",
  "term_id": "GO:0005667",
  "term_label": "transcription regulator complex",
  "gene_name": "Zinc finger protein 541",
  "gene": "UniProtKB:Q9H0D2"
}